{
  "term_id": "GO:0005730",
  "gene_name": "Dual specificity protein phosphatase CDC14C",
  "gene": "UniProtKB:A4D256",
  "term_label": "nucleolus",
  "gene_symbol": "CDC14C"
}